beta-mannosylphosphodecaprenol-mannooligosaccharide 6-mannosyltransferase activity [GO:0047252] (molecular function) Relationships: is a type of mannosyltransferase activity [GO:0000030] Definition: Catalysis of the reaction: (1->6)-alpha-D-mannosyloligosaccharide + beta-D-mannosylphosphodecaprenol = (1->6)-alpha-D-mannosyl-(1->6)-alpha-D-mannosyl-oligosaccharide + decaprenol phosphate. Also known as: beta-D-mannosylphosphodecaprenol:1,6-alpha-D-mannosyloligosaccharide 1,6-alpha-D-mannosyltransferase activity, mannosylphospholipid-methylmannoside alpha-1,6-mannosyltransferase activity Sources: EC:2.4.1.199, MetaCyc:2.4.1.199-RXN